{
  "gene_symbol": "ACTA1",
  "gene_name": "Actin, alpha skeletal muscle",
  "gene": "UniProtKB:P68133",
  "term_id": "GO:0015629",
  "term_label": "actin cytoskeleton"
}